{
  "term_id": "GO:0005634",
  "term_label": "nucleus",
  "gene_name": "Zinc finger protein 653",
  "gene_symbol": "ZNF653",
  "gene": "UniProtKB:Q96CK0"
}